{
  "gene_symbol": "REX1BD",
  "term_label": "Unknown cellular component",
  "gene": "UniProtKB:Q96EN9",
  "gene_name": "Required for excision 1-B domain-containing protein",
  "term_id": "UNKNOWN:0003"
}